{
  "term_label": "ubiquitin protein ligase activity",
  "gene_symbol": "TRIM26",
  "gene": "UniProtKB:Q12899",
  "gene_name": "Tripartite motif-containing protein 26",
  "term_id": "GO:0061630"
}